{
  "term_label": "neuronal cell body",
  "term_id": "GO:0043025",
  "gene_name": "Microtubule-associated protein 1A",
  "gene": "UniProtKB:P78559",
  "gene_symbol": "MAP1A"
}